{
  "gene": "UniProtKB:Q9BWH2",
  "gene_name": "FUN14 domain-containing protein 2",
  "term_label": "Unknown molecular function",
  "term_id": "UNKNOWN:0001",
  "gene_symbol": "FUNDC2"
}